{
  "term_id": "GO:0005886",
  "gene_name": "Transient receptor potential cation channel subfamily V member 5",
  "gene": "UniProtKB:Q9NQA5",
  "gene_symbol": "TRPV5",
  "term_label": "plasma membrane"
}